phototransduction, UV [GO:0007604] (biological process) Also known as: phototransduction, UV light, phototransduction, UV radiation, phototransduction, ultraviolet light, phototransduction, ultraviolet radiation, UV-sensitive opsin Sources: GOC:go_curators, ISBN:0198506732 Definition: The sequence of reactions within a cell required to convert absorbed photons from UV light into a molecular signal; ultraviolet radiation is electromagnetic radiation with a wavelength in the range of 10 to 400 nanometers. Relationships: is a type of GO:0007602; is a type of detection of UV [GO:0009589]; is a type of GO:0034644